{
  "term_label": "ATP metabolic process",
  "gene_name": "Ectonucleotide pyrophosphatase_phosphodiesterase family member 1",
  "gene": "UniProtKB:P22413",
  "gene_symbol": "ENPP1",
  "term_id": "GO:0046034"
}